{
  "term_id": "GO:0070888",
  "gene_symbol": "NEUROD4",
  "gene": "UniProtKB:Q9HD90",
  "term_label": "E-box binding",
  "gene_name": "Neurogenic differentiation factor 4"
}